protein-phosphocysteine-D-fructose-phosphotransferase system transporter activity [GO:0090582] (molecular function) References: PMID:8626640 Relationships: is a type of protein-phosphocysteine-sugar phosphotransferase activity [GO:0090563] Definition: Catalysis of the PEP-dependent, phosphoryl transfer-driven transport of substances across a membrane. The transport happens by catalysis of the reaction: protein S-phosphocysteine + D-fructose(out) = protein cysteine + D-fructose-1-phosphate(in).